{
  "gene": "UniProtKB:Q9BQB6",
  "term_id": "GO:0007596",
  "gene_symbol": "VKORC1",
  "term_label": "blood coagulation",
  "gene_name": "Vitamin K epoxide reductase complex subunit 1"
}